O-acetyl-ADP-ribose deacetylase activity [GO:0061463] (molecular function) Relationships: is a type of deacetylase activity [GO:0019213]; is a type of carboxylic ester hydrolase activity [GO:0052689] Definition: Catalysis of the reaction O-acetyl-ADP-ribose + H2O = ADP-ribose + acetate. Removes the acetyl group from either the 2'' or 3'' position of O-acetyl-ADP-ribose. Sources: EC:3.1.1.106